{
  "term_id": "GO:0005634",
  "gene": "UniProtKB:Q9NR09",
  "gene_name": "Baculoviral IAP repeat-containing protein 6",
  "gene_symbol": "BIRC6",
  "term_label": "nucleus"
}